{
  "gene_name": "Sterol carrier protein 2",
  "term_label": "Unknown biological process",
  "gene_symbol": "SCP2",
  "gene": "UniProtKB:P22307",
  "term_id": "UNKNOWN:0002"
}